neutrophil-mediated killing of gram-negative bacterium [GO:0070945] (biological process) Definition: The directed killing of a gram-negative bacterium by a neutrophil. Regulation: regulated by regulation of neutrophil mediated killing of gram-negative bacterium [GO:0070951]; negatively regulated by negative regulation of neutrophil mediated killing of gram-negative bacterium [GO:0070957]; positively regulated by positive regulation of neutrophil mediated killing of gram-negative bacterium [GO:0070963] Also known as: neutrophil mediated killing of gram-negative bacterium Relationships: is a type of neutrophil-mediated killing of bacterium [GO:0070944]; is part of defense response to Gram-negative bacterium [GO:0050829] Sources: GOC:add, ISBN:0781765196